{
  "gene_symbol": "DDX39A",
  "gene": "UniProtKB:O00148",
  "gene_name": "ATP-dependent RNA helicase DDX39A",
  "term_id": "GO:0003729",
  "term_label": "mRNA binding"
}